{
  "term_id": "GO:0005576",
  "gene": "UniProtKB:Q12841",
  "gene_symbol": "FSTL1",
  "gene_name": "Follistatin-related protein 1",
  "term_label": "extracellular region"
}